{
  "gene": "UniProtKB:P05089",
  "term_label": "manganese ion binding",
  "term_id": "GO:0030145",
  "gene_symbol": "ARG1",
  "gene_name": "Arginase-1"
}